invertasome [GO:0031421] (cellular component) Relationships: is a type of intracellular protein-containing complex [GO:0140535]; is a type of GO:1902494 References: PMID:11114897, PMID:9732277 Definition: A complex formed by a recombinase, a regulatory protein, and the DNA sequences bound by each protein; catalyzes a reversible site-specific recombination reaction that results in the alternate expression of one or more genes in various contexts.